{
  "gene_symbol": "ENOX2",
  "term_id": "UNKNOWN:0002",
  "gene_name": "Ecto-NOX disulfide-thiol exchanger 2",
  "term_label": "Unknown biological process",
  "gene": "UniProtKB:Q16206"
}